{
  "gene": "UniProtKB:Q9UMR7",
  "term_id": "GO:0030246",
  "gene_symbol": "CLEC4A",
  "term_label": "carbohydrate binding",
  "gene_name": "C-type lectin domain family 4 member A"
}